{
  "term_id": "GO:0000981",
  "term_label": "DNA-binding transcription factor activity, RNA polymerase II-specific",
  "gene": "UniProtKB:Q6NSW7",
  "gene_name": "Homeobox protein NANOGP8",
  "gene_symbol": "NANOGP8"
}